NAD-dependent protein-lysine depropionylase activity [GO:0106231] (MF) Note: This reaction is the removal of a propionyl group from a propionylated lysine residue of a protein or peptide. Relationships: is a type of NAD-dependent protein lysine deacylase activity [GO:0141218] References: PMID:30026585 Sources: GOC:sp, RHEA:23500 Definition: Catalysis of the reaction:H2O + N(6)-propanoyl-L-lysyl-[protein] + NAD+ = 3''-O-propanoyl-ADP-D-ribose + L-lysyl-[protein] + nicotinamide.